{
  "gene_symbol": "CYTL1",
  "term_label": "Unknown cellular component",
  "term_id": "UNKNOWN:0003",
  "gene_name": "Cytokine-like protein 1",
  "gene": "UniProtKB:Q9NRR1"
}